{
  "gene": "UniProtKB:Q9GZU3",
  "term_id": "UNKNOWN:0001",
  "gene_symbol": "TMEM39B",
  "term_label": "Unknown molecular function",
  "gene_name": "Transmembrane protein 39B"
}